{
  "term_id": "GO:0045095",
  "gene_symbol": "KRT5",
  "gene_name": "Keratin, type II cytoskeletal 5",
  "term_label": "keratin filament",
  "gene": "UniProtKB:P13647"
}